{
  "term_label": "brush border membrane",
  "gene": "UniProtKB:P48764",
  "term_id": "GO:0031526",
  "gene_symbol": "SLC9A3",
  "gene_name": "Sodium_hydrogen exchanger 3"
}